{
  "gene_symbol": "CEP89",
  "gene": "UniProtKB:Q96ST8",
  "term_label": "ciliary transition fiber",
  "gene_name": "Centrosomal protein of 89 kDa",
  "term_id": "GO:0097539"
}